{
  "term_id": "UNKNOWN:0003",
  "term_label": "Unknown cellular component",
  "gene_symbol": "TMEM200C",
  "gene": "UniProtKB:A6NKL6",
  "gene_name": "Transmembrane protein 200C"
}